{
  "term_label": "galactose 3-O-sulfotransferase activity",
  "gene_name": "Galactose-3-O-sulfotransferase 4",
  "term_id": "GO:0050694",
  "gene_symbol": "GAL3ST4",
  "gene": "UniProtKB:Q96RP7"
}